{
  "gene": "UniProtKB:O43482",
  "gene_symbol": "OIP5",
  "term_id": "GO:0000775",
  "gene_name": "Protein Mis18-beta",
  "term_label": "chromosome, centromeric region"
}